{
  "gene": "UniProtKB:Q9BWH6",
  "term_id": "UNKNOWN:0001",
  "gene_name": "RNA polymerase II-associated protein 1",
  "term_label": "Unknown molecular function",
  "gene_symbol": "RPAP1"
}